Flemming body [GO:0090543] (cellular component) Relationships: is a type of cellular anatomical structure [GO:0110165]; is part of midbody [GO:0030496] Also known as: Midbody ring Definition: A cell part that is the central region of the midbody characterized by a gap in alpha-tubulin staining. It is a dense structure of antiparallel microtubules from the central spindle in the middle of the intercellular bridge. References: PMID:18641129, PMID:22522702 Sources: GOC:pm